{
  "term_id": "UNKNOWN:0001",
  "gene": "UniProtKB:Q9UBQ0",
  "gene_name": "Vacuolar protein sorting-associated protein 29",
  "gene_symbol": "VPS29",
  "term_label": "Unknown molecular function"
}